{
  "gene_name": "E3 ubiquitin-protein ligase UBR5",
  "gene": "UniProtKB:O95071",
  "term_label": "protein polyubiquitination",
  "term_id": "GO:0000209",
  "gene_symbol": "UBR5"
}